fatty acid derivative binding [GO:1901567] (molecular function) Subtypes: fatty-acyl-CoA binding [GO:0000062], 5-hydroxy-6E,8Z,11Z,14Z-icosatetraenoic acid binding [GO:0050647], GO:0050648, prostaglandin binding [GO:1904593] Relationships: is a type of lipid binding [GO:0008289] Definition: Binding to fatty acid derivative. Sources: GOC:TermGenie, GOC:pr